myosin X complex [GO:0031480] (cellular component) Definition: A myosin complex containing one or more class X myosin heavy chains and associated light chains. Relationships: is a type of GO:0016461 References: PMID:27580874 Sources: https://doi.org/10.9729/AM.2018.48.2.33